{
  "term_id": "UNKNOWN:0003",
  "gene": "UniProtKB:Q14602",
  "term_label": "Unknown cellular component",
  "gene_symbol": "ID2B",
  "gene_name": "Putative DNA-binding protein inhibitor ID-2B"
}